alphaV-beta6 integrin-osteopontin complex [GO:0071126] (cellular component) References: PMID:16005200 Definition: A protein complex that consists of an alphaV-beta6 integrin complex bound to osteopontin. Relationships: is a type of plasma membrane protein complex [GO:0098797] Also known as: ITGAV-ITGB6-SPP1 complex